{
  "gene_symbol": "ZNF230",
  "term_label": "Unknown cellular component",
  "gene_name": "Zinc finger protein 230",
  "term_id": "UNKNOWN:0003",
  "gene": "UniProtKB:Q9UIE0"
}